AMP catabolic process [GO:0006196] (biological process) Definition: The chemical reactions and pathways resulting in the breakdown of AMP, adenosine monophosphate. Sources: ISBN:0198506732 Also known as: AMP breakdown, AMP catabolism, AMP degradation Relationships: is a type of purine ribonucleotide catabolic process [GO:0009154]; is a type of purine ribonucleoside monophosphate catabolic process [GO:0009169]; is a type of GO:0046033